{
  "gene_symbol": "GATAD2B",
  "gene_name": "Transcriptional repressor p66-beta",
  "gene": "UniProtKB:Q8WXI9",
  "term_id": "GO:0000122",
  "term_label": "negative regulation of transcription by RNA polymerase II"
}